silver ion transmembrane transporter complex [GO:1903114] (cellular component) Definition: A protein complex which is capable of silver ion transmembrane transporter activity. References: PMID:11283292 Sources: GOC:TermGenie, GOC:bhm, GO_REF:0000088 Note: An example of this is CusA in E. coli (UniProt symbol P38054) in PMID:11283292 (inferred from direct assay). Relationships: is_a transmembrane transporter complex [GO:1902495] Subtypes: Cus cation efflux complex [GO:1990398]